glyceraldehyde-3-phosphate dehydrogenase (NAD+) (phosphorylating) activity [GO:0004365] (molecular function) Relationships: is a type of glyceraldehyde-3-phosphate dehydrogenase [NAD(P)+] (phosphorylating) activity [GO:0043891] Also known as: triosephosphate dehydrogenase activity, 3-phosphoglyceraldehyde dehydrogenase activity, D-glyceraldehyde-3-phosphate:NAD+ oxidoreductase (phosphorylating), GAPDH activity, NAD-dependent glyceraldehyde phosphate dehydrogenase activity, NAD-dependent glyceraldehyde-3-phosphate dehydrogenase activity, NADH-glyceraldehyde phosphate dehydrogenase activity, dehydrogenase, glyceraldehyde phosphate, glyceraldehyde phosphate dehydrogenase (NAD), glyceraldehyde-3-P-dehydrogenase activity, phosphoglyceraldehyde dehydrogenase activity Sources: EC:1.2.1.12 Definition: Catalysis of the reaction: D-glyceraldehyde 3-phosphate + phosphate + NAD+ = 3-phospho-D-glyceroyl phosphate + NADH + H+.